pentacyclic triterpenoid metabolic process [GO:0019742] (biological process) Definition: The chemical reactions and pathways involving pentacyclic triterpenoid compounds, terpenoids with six isoprene units and 5 carbon rings. Sources: ISBN:0198506732 Also known as: pentacyclic triterpenoid metabolism Relationships: is_a triterpenoid metabolic process [GO:0006722] Subtypes: pentacyclic triterpenoid catabolic process [GO:0019741], pentacyclic triterpenoid biosynthetic process [GO:0019745]